regulation of positive chemotaxis to cAMP by DIF-1 [GO:0061120] (BP) Subtypes: GO:0061126, negative regulation of positive chemotaxis to cAMP by DIF-1 [GO:0061127] Sources: GOC:dph Definition: Any process that modulates the rate, frequency, or extent of directed movement of a motile cell or organism up a concentration gradient of 3',5'-cAMP by the action of DIF-1. DIF-1 is a chlorinated alkylphenone. Relationships: is a type of regulation of positive chemotaxis to cAMP by chlorinated alkylphenone [GO:0061119]